{
  "term_label": "natural killer cell activation involved in immune response",
  "term_id": "GO:0002323",
  "gene_symbol": "IFNK",
  "gene": "UniProtKB:Q9P0W0",
  "gene_name": "Interferon kappa"
}